{
  "gene": "UniProtKB:Q6ZUV0",
  "term_id": "GO:0005829",
  "gene_symbol": "ACOT7L",
  "gene_name": "Putative cytosolic acyl coenzyme A thioester hydrolase-like",
  "term_label": "cytosol"
}